regulation of signal transduction by receptor internalization [GO:0038009] (biological process) Relationships: is a type of regulation of signal transduction [GO:0009966]; is a type of receptor internalization [GO:0031623] References: PMID:17011816, PMID:19696798 Sources: GOC:bf, GOC:signaling Definition: Any process that modulates the frequency, rate or extent of signal transduction by the movement of a signaling receptor from the plasma membrane to the inside of the cell. Receptor internalization can have a positive or negative effect on a signaling pathway. Subtypes: GO:0038010, negative regulation of signal transduction by receptor internalization [GO:0038011] Also known as: regulation of signaling pathway by receptor endocytosis